{
  "term_id": "GO:0032570",
  "gene_name": "Alpha-S1-casein",
  "gene": "UniProtKB:P47710",
  "gene_symbol": "CSN1S1",
  "term_label": "response to progesterone"
}